{
  "term_id": "UNKNOWN:0003",
  "gene_symbol": "MINAR2",
  "gene": "UniProtKB:P59773",
  "gene_name": "Major intrinsically disordered NOTCH2-binding receptor 1-like",
  "term_label": "Unknown cellular component"
}